{
  "term_id": "UNKNOWN:0003",
  "term_label": "Unknown cellular component",
  "gene": "UniProtKB:B2RD01",
  "gene_symbol": "CENPBD1P",
  "gene_name": "Putative CENPB DNA-binding domain-containing protein 1"
}